{
  "term_id": "GO:0005634",
  "gene_symbol": "ZXDC",
  "gene_name": "Zinc finger protein ZXDC",
  "term_label": "nucleus",
  "gene": "UniProtKB:Q2QGD7"
}